{
  "gene_symbol": "MIER1",
  "term_label": "negative regulation of transcription by RNA polymerase II",
  "gene": "UniProtKB:Q8N108",
  "term_id": "GO:0000122",
  "gene_name": "Mesoderm induction early response protein 1"
}